{
  "gene_name": "E3 ubiquitin-protein ligase SIAH1",
  "gene": "UniProtKB:Q8IUQ4",
  "term_id": "GO:0031624",
  "gene_symbol": "SIAH1",
  "term_label": "ubiquitin conjugating enzyme binding"
}